vacuolar HOPS complex [GO:1902500] (cellular component) Relationships: is a type of HOPS complex [GO:0030897]; is part of vacuolar membrane [GO:0005774] Subtypes: lysosomal HOPS complex [GO:1902501] Also known as: vacuolar membrane HOPS complex Definition: Any HOPS complex that is part of a vacuolar membrane. References: PMID:23645161 Sources: GOC:TermGenie